glycine N-acyltransferase activity [GO:0047961] (MF) Definition: Catalysis of the reaction: acyl-CoA + glycine = CoA + N-acylglycine. Also known as: acyl-CoA:glycine N-acyltransferase activity, glycine acyltransferase activity, glycine-N-acylase activity Sources: EC:2.3.1.13, MetaCyc:GLYCINE-N-ACYLTRANSFERASE-RXN Relationships: is a type of GO:0016410